{
  "term_label": "triglyceride mobilization",
  "term_id": "GO:0006642",
  "gene_name": "Apolipoprotein B-100",
  "gene": "UniProtKB:P04114",
  "gene_symbol": "APOB"
}